{
  "term_id": "GO:0140912",
  "gene": "UniProtKB:Q30KP9",
  "gene_name": "Beta-defensin 135",
  "gene_symbol": "DEFB135",
  "term_label": "membrane destabilizing activity"
}